{
  "gene_name": "Inhibitor of Bruton tyrosine kinase",
  "gene_symbol": "IBTK",
  "gene": "UniProtKB:Q9P2D0",
  "term_label": "release of sequestered calcium ion into cytosol",
  "term_id": "GO:0051209"
}